glial cell-derived neurotrophic factor receptor signaling pathway [GO:0035860] (biological process) Definition: The series of molecular signals initiated by a ligand binding to a glial cell-derived neurotrophic factor receptor. Also known as: GDNF receptor signaling pathway, glial cell derived neurotrophic factor receptor signaling pathway, glial cell line-derived neurotrophic factor receptor signalling pathway, glial cell-derived neurotrophic factor receptor signalling pathway References: PMID:12953054, PMID:29245123 Sources: GOC:yaf Subtypes: GDF15-GFRAL signaling pathway [GO:0160144], glial cell-derived neurotrophic factor receptor signaling pathway involved in ureteric bud formation [GO:2000701] Relationships: is a type of GO:0007169